{
  "gene_name": "Collagen alpha-2(V) chain",
  "gene": "UniProtKB:P05997",
  "gene_symbol": "COL5A2",
  "term_id": "GO:0030020",
  "term_label": "extracellular matrix structural constituent conferring tensile strength"
}